1,2,3-tribromopropane metabolic process [GO:0018976] (biological process) Definition: The chemical reactions and pathways involving 1,2,3-tribromopropane, a toxic and volatile organic compound commonly used as a nematocide in agriculture. Sources: GOC:jl Also known as: 1,2,3-tribromopropane metabolism Relationships: is_a halogenated hydrocarbon metabolic process [GO:0042197]